{
  "term_label": "transmembrane transport",
  "gene_name": "Proton-coupled folate transporter",
  "term_id": "GO:0055085",
  "gene_symbol": "SLC46A1",
  "gene": "UniProtKB:Q96NT5"
}